borate binding [GO:0046714] (molecular function) Sources: GOC:curators Also known as: boron binding Definition: Binding to borate, the anion (BO3)3-. Relationships: is a type of anion binding [GO:0043168]